{
  "gene": "UniProtKB:Q9BT09",
  "gene_name": "Protein canopy homolog 3",
  "term_label": "signaling receptor binding",
  "gene_symbol": "CNPY3",
  "term_id": "GO:0005102"
}